mesonephric glomerulus morphogenesis [GO:0061234] (biological process) Definition: The process in which the anatomical structures of the mesonephric glomerulus are generated and organized. The mesonephric glomerulus is a capillary tuft surrounded by Bowman's capsule in nephrons of the vertebrate mesonephros. Sources: GOC:mtg_kidney_jan10 Relationships: is a type of glomerulus morphogenesis [GO:0072102]; is part of mesonephric glomerulus development [GO:0061224]; is part of mesonephric nephron morphogenesis [GO:0061228]